{
  "term_label": "sodium ion transmembrane transport",
  "term_id": "GO:0035725",
  "gene_name": "Sodium- and chloride-dependent neutral and basic amino acid transporter B(0+)",
  "gene_symbol": "SLC6A14",
  "gene": "UniProtKB:Q9UN76"
}